{
  "term_id": "GO:0003823",
  "gene_name": "Immunoglobulin heavy variable 1_OR15-1 (non-functional) (Fragment)",
  "gene_symbol": "IGHV1OR15-1",
  "term_label": "antigen binding",
  "gene": "UniProtKB:A0A075B7D0"
}